conidiophore stalk development [GO:0070788] (biological process) Relationships: is a type of GO:0003006; is a type of anatomical structure development [GO:0048856]; is part of conidiophore development [GO:0070787] References: PMID:9529886 Definition: The process whose specific outcome is the progression of the conidiophore stalk over time, from its formation to the mature structure. The conidiophore stalk is part of a specialized hypha that extends aerially from the growth substrate and supports structures from which conidia, or asexual spores, develop. Regulation: regulated by regulation of conidiophore stalk development [GO:0070799]; negatively regulated by negative regulation of conidiophore stalk development [GO:0070800]; positively regulated by positive regulation of conidiophore stalk development [GO:0070801]